{
  "term_label": "Unknown cellular component",
  "term_id": "UNKNOWN:0003",
  "gene_name": "Putative uncharacterized protein SNHG28",
  "gene": "UniProtKB:P0DPA3",
  "gene_symbol": "SNHG28"
}